{
  "gene": "UniProtKB:A0A1B0GW15",
  "term_id": "UNKNOWN:0001",
  "gene_symbol": "LOC122394732",
  "term_label": "Unknown molecular function",
  "gene_name": "Uncharacterized protein"
}